N-acetylglucosamine-1-phosphodiester alpha-N-acetylglucosaminidase activity [GO:0003944] (molecular function) Relationships: is a type of GO:0015929 Sources: EC:3.1.4.45 Definition: Catalysis of the reaction: glycoprotein N-acetyl-D-glucosaminyl-phospho-D-mannose + H2O = N-acetyl-D-glucosamine + glycoprotein phospho-D-mannose. Also known as: lysosomal alpha-N-acetylglucosaminidase activity, 2-acetamido-2-deoxy-alpha-D-glucose 1-phosphodiester acetamidodeoxyglucohydrolase activity, alpha-N-acetyl-D-glucosamine-1-phosphodiester N-acetylglucosaminidase activity, alpha-N-acetylglucosaminyl phosphodiesterase activity, glycoprotein-N-acetyl-D-glucosaminyl-phospho-D-mannose N-acetyl-D-glucosaminylphosphohydrolase activity, phosphodiester glycosidase activity